{
  "gene": "UniProtKB:Q9UHF4",
  "term_label": "cytokine receptor activity",
  "gene_name": "Interleukin-20 receptor subunit alpha",
  "gene_symbol": "IL20RA",
  "term_id": "GO:0004896"
}